1-deoxy-D-xylulose kinase activity [GO:0103020] (molecular function) References: PMID:11168365, PMID:16920870 Sources: GOC:pz Definition: Catalysis of the reaction: 1-deoxy-D-xylulose + ATP = H+ + 1-deoxy-D-xylulose 5-phosphate + ADP. Relationships: is a type of phosphotransferase activity, alcohol group as acceptor [GO:0016773]